{
  "gene_name": "Glutathione S-transferase theta-1",
  "term_label": "glutathione metabolic process",
  "term_id": "GO:0006749",
  "gene_symbol": "GSTT1",
  "gene": "UniProtKB:P30711"
}